CXCR4 chemokine receptor binding [GO:0031723] (molecular function) Relationships: is a type of CXCR chemokine receptor binding [GO:0045236] Also known as: stromal cell-derived factor 1 receptor binding, CXCR4 chemokine receptor ligand Sources: GOC:mah, GOC:nln Definition: Binding to a CXCR4 chemokine receptor.